{
  "gene": "UniProtKB:Q9H4S2",
  "gene_name": "GS homeobox 1",
  "term_id": "GO:0007417",
  "term_label": "central nervous system development",
  "gene_symbol": "GSX1"
}